{
  "gene_symbol": "IFT70A",
  "term_label": "intraciliary transport particle B",
  "term_id": "GO:0030992",
  "gene_name": "Intraflagellar transport protein 70A",
  "gene": "UniProtKB:Q86WT1"
}